negative regulation of eosinophil activation [GO:1902567] (biological process) Definition: Any process that stops, prevents or reduces the frequency, rate or extent of eosinophil activation. References: PMID:16254138 Sources: GOC:TermGenie Also known as: down regulation of eosinophil activation, down-regulation of eosinophil activation, downregulation of eosinophil activation, inhibition of eosinophil activation Relationships: is_a negative regulation of leukocyte activation [GO:0002695]; is a type of regulation of eosinophil activation [GO:1902566]; RO_0002212 eosinophil activation [GO:0043307]